{
  "term_label": "cysteine-type endopeptidase inhibitor activity",
  "gene": "UniProtKB:O76096",
  "term_id": "GO:0004869",
  "gene_name": "Cystatin-F",
  "gene_symbol": "CST7"
}